quinone reductase (NADPH) activity [GO:0003960] (MF) Definition: Catalysis of the reaction: 2 a quinone + NADPH + H+ = 2 a 1,4-benzosemiquinone + NADP+. Sources: RHEA:14269 Also known as: quinone oxidoreductase activity, NADPH:quinone reductase activity, zeta-crystallin activity, NADPH:quinone oxidoreductase activity Relationships: is a type of GO:0003959; is_a oxidoreductase activity, acting on NAD(P)H, quinone or similar compound as acceptor [GO:0016655]